{
  "gene": "UniProtKB:O95070",
  "term_id": "GO:0006888",
  "gene_symbol": "YIF1A",
  "term_label": "endoplasmic reticulum to Golgi vesicle-mediated transport",
  "gene_name": "Protein YIF1A"
}